{
  "gene_name": "Platelet glycoprotein IX",
  "gene": "UniProtKB:P14770",
  "term_id": "UNKNOWN:0001",
  "gene_symbol": "GP9",
  "term_label": "Unknown molecular function"
}